{
  "term_id": "GO:0003714",
  "gene_name": "Metastasis-associated protein MTA2",
  "gene_symbol": "MTA2",
  "term_label": "transcription corepressor activity",
  "gene": "UniProtKB:O94776"
}